threo-3-hydroxyaspartate ammonia-lyase activity [GO:0030848] (molecular function) Definition: Catalysis of the reaction: (3S)-3-hydroxy-L-aspartate = NH4 + oxaloacetate. Sources: EC:4.3.1.16, RHEA:12424 Also known as: 3-hydroxyaspartate dehydratase activity, L-threo-3-hydroxyaspartate dehydratase activity, threo-3-hydroxy-L-aspartate ammonia-lyase (oxaloacetate-forming), threo-3-hydroxy-L-aspartate ammonia-lyase activity, threo-3-hydroxyaspartate dehydratase activity Relationships: is a type of GO:0016841